mannose isomerase activity [GO:0050089] (molecular function) Also known as: D-mannose aldose-ketose-isomerase activity, D-mannose isomerase activity, D-mannose ketol-isomerase activity Relationships: is a type of GO:0016861 Sources: RHEA:22604 Definition: Catalysis of the reaction: D-mannose = D-fructose.